{
  "term_id": "GO:0071011",
  "gene_symbol": "SNRPG",
  "gene": "UniProtKB:P62308",
  "gene_name": "Small nuclear ribonucleoprotein G",
  "term_label": "precatalytic spliceosome"
}